{
  "gene_name": "Interferon regulatory factor 6",
  "gene_symbol": "IRF6",
  "term_id": "GO:0005634",
  "term_label": "nucleus",
  "gene": "UniProtKB:O14896"
}